{
  "term_id": "GO:0016891",
  "gene": "UniProtKB:Q8N8Q3",
  "term_label": "RNA endonuclease activity producing 5'-phosphomonoesters, hydrolytic mechanism",
  "gene_symbol": "ENDOV",
  "gene_name": "Endonuclease V"
}